estrogen receptor signaling pathway [GO:0030520] (biological process) Definition: A nuclear receptor-mediated signaling pathway initiated by an estrogen binding to an intracellular receptor of the nuclear receptor protein family, and ending with regulation of a downstream cellular process, e.g. transcription. Also known as: estrogen receptor signalling pathway, intracellular estrogen receptor signaling pathway, nuclear receptor-mediated estrogen signaling pathway Regulation: RO_0002211 by regulation of intracellular estrogen receptor signaling pathway [GO:0033146]; negatively regulated by negative regulation of intracellular estrogen receptor signaling pathway [GO:0033147]; RO_0002213 by positive regulation of intracellular estrogen receptor signaling pathway [GO:0033148] Sources: GOC:signaling Relationships: is a type of nuclear receptor-mediated steroid hormone signaling pathway [GO:0030518]